cytosolic mRNA polyadenylation [GO:0180011] (biological process) Relationships: is a type of mRNA metabolic process [GO:0016071] References: PMID:21536428 Definition: Any process by which dormant, translationally inactive mRNAs become activated, or mRNAs become stabilized, via the elongation of their poly(A) tails in the cytosol.